phosphatidylglycerol catabolic process [GO:0034478] (BP) Definition: The chemical reactions and pathways resulting in the breakdown of phosphatidylglycerols, any of a class of glycerophospholipids in which the phosphatidyl group is esterified to the hydroxyl group of glycerol. Relationships: is a type of phosphatidylglycerol metabolic process [GO:0046471]; is a type of glycerophospholipid catabolic process [GO:0046475] Also known as: phosphatidylglycerol breakdown, phosphatidylglycerol catabolism, phosphatidylglycerol degradation Sources: GOC:mah